{
  "gene_symbol": "TTC32",
  "term_label": "Unknown molecular function",
  "gene_name": "Tetratricopeptide repeat protein 32",
  "gene": "UniProtKB:Q5I0X7",
  "term_id": "UNKNOWN:0001"
}